{
  "gene": "UniProtKB:P04035",
  "term_label": "endoplasmic reticulum membrane",
  "gene_name": "3-hydroxy-3-methylglutaryl-coenzyme A reductase",
  "term_id": "GO:0005789",
  "gene_symbol": "HMGCR"
}